{
  "gene": "UniProtKB:O43295",
  "term_id": "GO:0005096",
  "term_label": "GTPase activator activity",
  "gene_symbol": "SRGAP3",
  "gene_name": "SLIT-ROBO Rho GTPase-activating protein 3"
}